metal cluster binding [GO:0051540] (MF) Sources: GOC:jsg Definition: Binding to a cluster of atoms including both metal ions and nonmetal atoms, usually sulfur and oxygen. Examples include iron-sulfur clusters and nickel-iron-sulfur clusters. Relationships: is_a GO:0036094 Subtypes: dinitrosyl-iron complex binding [GO:0035731], iron-sulfur cluster binding [GO:0051536]